{
  "gene_name": "Protein-glutamine gamma-glutamyltransferase K",
  "gene_symbol": "TGM1",
  "term_label": "peptide cross-linking",
  "term_id": "GO:0018149",
  "gene": "UniProtKB:P22735"
}